negative regulation of erythrophore differentiation [GO:0048779] (biological process) Also known as: down regulation of erythrophore differentiation, down-regulation of erythrophore differentiation, downregulation of erythrophore differentiation, inhibition of erythrophore differentiation Definition: Any process that stops, prevents, or reduces the frequency, rate or extent of erythrophore differentiation. Relationships: is a type of GO:0048778; is a type of GO:0050941; negatively regulates erythrophore differentiation [GO:0048773] Sources: GOC:mh